response to catecholamine [GO:0071869] (biological process) Also known as: response to catecholamine stimulus Sources: GOC:BHF, GOC:mah Definition: Any process that results in a change in state or activity of a cell or an organism (in terms of movement, secretion, enzyme production, gene expression, etc.) as a result of a catecholamine stimulus. A catecholamine is any of a group of biogenic amines that includes 4-(2-aminoethyl)pyrocatechol [4-(2-aminoethyl)benzene-1,2-diol] and derivatives formed by substitution. Subtypes: GO:0071870, response to norepinephrine [GO:0071873], GO:1903350, response to oxidopamine [GO:1905841] Relationships: is a type of response to monoamine [GO:0071867]; is a type of response to oxygen-containing compound [GO:1901700]